muramyl dipeptide binding [GO:0032500] (MF) Sources: GOC:rl Relationships: is a type of amide binding [GO:0033218]; is a type of monocarboxylic acid binding [GO:0033293]; is a type of carbohydrate derivative binding [GO:0097367] Definition: Interacting selectively and non-covalently, in a non-covalent manner, with muramyl dipeptide; muramyl dipeptide is derived from peptidoglycan.